{
  "gene_name": "Regulator of MON1-CCZ1 complex",
  "gene_symbol": "RMC1",
  "term_id": "GO:0035658",
  "gene": "UniProtKB:Q96DM3",
  "term_label": "Mon1-Ccz1 complex"
}